{
  "gene": "UniProtKB:P05067",
  "gene_name": "Amyloid-beta precursor protein",
  "gene_symbol": "APP",
  "term_label": "Golgi apparatus",
  "term_id": "GO:0005794"
}